{
  "term_label": "macrophage activation involved in immune response",
  "gene_name": "Protein strawberry notch homolog 2",
  "gene_symbol": "SBNO2",
  "gene": "UniProtKB:Q9Y2G9",
  "term_id": "GO:0002281"
}